{
  "gene_symbol": "SNED1",
  "term_id": "UNKNOWN:0002",
  "term_label": "Unknown biological process",
  "gene": "UniProtKB:Q8TER0",
  "gene_name": "Sushi, nidogen and EGF-like domain-containing protein 1"
}